tRNA 5'-end processing [GO:0099116] (biological process) Relationships: is a type of GO:0000966; is a type of GO:0008033 References: PMID:27484477 Sources: GOC:dos, GOC:pf Definition: The process in which the 5' end of a pre-tRNA molecule is converted to that of a mature tRNA. Subtypes: tRNA 5'-leader removal [GO:0001682], mitochondrial tRNA 5'-end processing [GO:0097745] Also known as: tRNA 5' processing